{
  "gene_symbol": "TMEM225B",
  "term_id": "UNKNOWN:0001",
  "term_label": "Unknown molecular function",
  "gene_name": "Transmembrane protein 225B",
  "gene": "UniProtKB:P0DP42"
}